{
  "gene_symbol": "ZGLP1",
  "gene_name": "GATA-type zinc finger protein 1",
  "term_id": "GO:0005634",
  "term_label": "nucleus",
  "gene": "UniProtKB:P0C6A0"
}